{
  "term_label": "nuclear export",
  "gene_name": "RanBP2-like and GRIP domain-containing protein 3",
  "gene_symbol": "RGPD3",
  "term_id": "GO:0051168",
  "gene": "UniProtKB:A6NKT7"
}